{
  "gene_name": "60S ribosome subunit biogenesis protein NIP7 homolog",
  "gene": "UniProtKB:Q9Y221",
  "gene_symbol": "NIP7",
  "term_id": "GO:0042273",
  "term_label": "ribosomal large subunit biogenesis"
}